{
  "gene_name": "Hypoxia-inducible factor 1-alpha inhibitor",
  "gene_symbol": "HIF1AN",
  "term_label": "[protein]-asparagine 3-dioxygenase activity",
  "term_id": "GO:0036140",
  "gene": "UniProtKB:Q9NWT6"
}